{
  "term_label": "chemical synaptic transmission",
  "gene_name": "Protein ELFN1",
  "term_id": "GO:0007268",
  "gene": "UniProtKB:P0C7U0",
  "gene_symbol": "ELFN1"
}